G-protein activated inward rectifier potassium channel activity [GO:0015467] (molecular function) Also known as: G protein activated inward rectifier potassium channel activity, G protein enhanced inward rectifier potassium channel activity, G-protein enhanced inward rectifier potassium channel activity, G-protein-activated inward rectifier potassium channel activity, G-protein-enhanced inward rectifier potassium channel activity Sources: GOC:cb, GOC:mah Definition: Enables the transmembrane transfer of a potassium ion by an inwardly-rectifying voltage-gated channel, where the inward rectification is due to a voltage-dependent block of the channel pore by a G protein. An inwardly rectifying current-voltage relation is one where at any given driving force the inward flow of K+ ions exceeds the outward flow for the opposite driving force. Relationships: is a type of GO:0005242